{
  "gene_name": "Guanine nucleotide exchange factor C9orf72",
  "gene": "UniProtKB:Q96LT7",
  "term_id": "GO:0005768",
  "term_label": "endosome",
  "gene_symbol": "C9orf72"
}